{
  "gene_name": "Histone H1.4",
  "gene_symbol": "H1-4",
  "term_label": "nucleosomal DNA binding",
  "term_id": "GO:0031492",
  "gene": "UniProtKB:P10412"
}